{
  "gene_name": "Tripartite motif-containing protein 44",
  "term_label": "innate immune response",
  "gene_symbol": "TRIM44",
  "gene": "UniProtKB:Q96DX7",
  "term_id": "GO:0045087"
}